regulation of BMP signaling pathway [GO:0030510] (biological process) Subtypes: GO:0030513, negative regulation of BMP signaling pathway [GO:0030514] Definition: Any process that modulates the frequency, rate or extent of the activity of any BMP receptor signaling pathway. Sources: GOC:mah Also known as: regulation of BMP signalling pathway, regulation of bone morphogenetic protein signaling pathway, regulation of bone morphogenetic protein signalling pathway, regulation of decapentaplegic receptor signaling pathway, regulation of decapentaplegic receptor signalling pathway, regulation of decapentaplegic signaling pathway, regulation of BMP receptor signaling pathway Relationships: is a type of GO:0090092; is_a regulation of cellular response to growth factor stimulus [GO:0090287]; regulates BMP signaling pathway [GO:0030509]